{
  "gene_name": "Heterogeneous nuclear ribonucleoprotein A3",
  "gene": "UniProtKB:P51991",
  "term_id": "GO:0071013",
  "gene_symbol": "HNRNPA3",
  "term_label": "catalytic step 2 spliceosome"
}